{
  "term_id": "GO:0005886",
  "gene": "UniProtKB:A0A0K0K1C4",
  "gene_symbol": "TRBV27",
  "term_label": "plasma membrane",
  "gene_name": "T cell receptor beta variable 27"
}